symbiont-mediated disruption of host cuticle [GO:0085044] (biological process) Relationships: is a type of symbiont-mediated disruption of host anatomical structure [GO:0052111] Also known as: catabolism of host cuticle, degradation of host cuticle, disassembly by symbiont of host cuticle Sources: GOC:jl, GOC:pamgo_curators Definition: The process in which an organism effects a change that impairs the structure or function of the host organism cuticle. The host is defined as the larger of the organisms involved in a symbiotic interaction.